{
  "gene": "UniProtKB:Q9UGP8",
  "term_label": "Sec62/Sec63 complex",
  "gene_symbol": "SEC63",
  "gene_name": "Translocation protein SEC63 homolog",
  "term_id": "GO:0031207"
}